vesicle scission [GO:0099050] (biological process) Definition: The membrane scission process that is the final step in the formation of a vesicle, leading to separation from its parent membrane. Vesicle scission involves the constriction of a neck-forming protein complex, consisting e.g. of dynamin, around the budded membrane, leading to vesicle closure during its separation from the parent membrane. References: PMID:21779028 Relationships: is a type of membrane fission [GO:0090148] Subtypes: vesicle scission involved in endocytosis [GO:0099051]